regulation of hexasaccharide transport [GO:1900297] (biological process) Definition: Any process that modulates the frequency, rate or extent of hexasaccharide transport. Subtypes: negative regulation of hexasaccharide transport [GO:1900298], positive regulation of hexasaccharide transport [GO:1900299], regulation of maltohexaose transport [GO:1900312] Sources: GOC:TermGenie, GOC:mengo_curators Relationships: is a type of regulation of transport [GO:0051049]; regulates GO:2001102